{
  "term_id": "GO:0006120",
  "gene_symbol": "NDUFA10",
  "gene_name": "NADH dehydrogenase [ubiquinone] 1 alpha subcomplex subunit 10, mitochondrial",
  "term_label": "mitochondrial electron transport, NADH to ubiquinone",
  "gene": "UniProtKB:O95299"
}